{
  "gene_name": "Trafficking protein particle complex subunit 1",
  "term_id": "GO:0006888",
  "gene_symbol": "TRAPPC1",
  "term_label": "endoplasmic reticulum to Golgi vesicle-mediated transport",
  "gene": "UniProtKB:Q9Y5R8"
}